{
  "term_id": "GO:0005886",
  "gene": "UniProtKB:P27930",
  "gene_name": "Interleukin-1 receptor type 2",
  "term_label": "plasma membrane",
  "gene_symbol": "IL1R2"
}